{
  "gene": "UniProtKB:Q5T3J3",
  "gene_name": "Ligand-dependent nuclear receptor-interacting factor 1",
  "term_label": "Unknown biological process",
  "term_id": "UNKNOWN:0002",
  "gene_symbol": "LRIF1"
}